4-hydroxyphenylacetate transmembrane transporter activity [GO:1901241] (MF) Relationships: is a type of monocarboxylic acid transmembrane transporter activity [GO:0008028] References: PMID:9315705 Sources: GOC:TermGenie Definition: Enables the transfer of 4-hydroxyphenylacetate from one side of a membrane to the other.